fibroblast apoptotic process [GO:0044346] (biological process) Definition: Any apoptotic process in a fibroblast, a connective tissue cell which secretes an extracellular matrix rich in collagen and other macromolecules. Also known as: fibroblast apoptosis Regulation: regulated by regulation of fibroblast apoptotic process [GO:2000269]; negatively regulated by negative regulation of fibroblast apoptotic process [GO:2000270]; RO_0002213 by GO:2000271 Relationships: is a type of apoptotic process [GO:0006915] Sources: CL:0000057, GOC:jl, GOC:mtg_apoptosis, GOC:yaf